{
  "gene": "UniProtKB:Q9HAT2",
  "term_label": "carbohydrate metabolic process",
  "gene_name": "Sialate O-acetylesterase",
  "term_id": "GO:0005975",
  "gene_symbol": "SIAE"
}